{
  "gene": "UniProtKB:Q86SE8",
  "term_label": "histone binding",
  "term_id": "GO:0042393",
  "gene_name": "Nucleoplasmin-2",
  "gene_symbol": "NPM2"
}